{
  "gene": "UniProtKB:P41226",
  "term_label": "DNA damage response",
  "gene_name": "Ubiquitin-like modifier-activating enzyme 7",
  "term_id": "GO:0006974",
  "gene_symbol": "UBA7"
}